{
  "gene": "UniProtKB:A6NHY2",
  "gene_name": "Ankyrin repeat and death domain-containing protein 1B",
  "term_label": "Unknown cellular component",
  "term_id": "UNKNOWN:0003",
  "gene_symbol": "ANKDD1B"
}